{
  "term_label": "autophagosome",
  "gene_name": "Ras-related protein Rab-24",
  "gene_symbol": "RAB24",
  "gene": "UniProtKB:Q969Q5",
  "term_id": "GO:0005776"
}